{
  "term_label": "Unknown cellular component",
  "term_id": "UNKNOWN:0003",
  "gene_symbol": "TMEM109",
  "gene_name": "Transmembrane protein 109",
  "gene": "UniProtKB:Q9BVC6"
}